{
  "term_id": "GO:0005886",
  "gene_name": "Hydroxycarboxylic acid receptor 2",
  "gene_symbol": "HCAR2",
  "gene": "UniProtKB:Q8TDS4",
  "term_label": "plasma membrane"
}